positive regulation of preblastoderm mitotic cell cycle [GO:0046002] (biological process) Relationships: is_a GO:0007347; is a type of positive regulation of mitotic cell cycle, embryonic [GO:0045977]; positively regulates GO:0035185 Also known as: positive regulation of preblastoderm mitotic cell cycle progression, positive regulation of progression through preblastoderm mitotic cell cycle, up regulation of progression through preblastoderm mitotic cell cycle, up-regulation of progression through preblastoderm mitotic cell cycle, upregulation of progression through preblastoderm mitotic cell cycle, activation of progression through preblastoderm mitotic cell cycle, stimulation of progression through preblastoderm mitotic cell cycle Sources: GOC:dph, GOC:go_curators, GOC:tb Definition: Any process that activates or increases the rate or extent of progression through the preblastoderm mitotic cell cycle.